{
  "term_id": "GO:0032456",
  "gene": "UniProtKB:Q9H223",
  "gene_symbol": "EHD4",
  "term_label": "endocytic recycling",
  "gene_name": "EH domain-containing protein 4"
}